{
  "gene": "UniProtKB:P58180",
  "gene_symbol": "OR4D2",
  "term_label": "plasma membrane",
  "gene_name": "Olfactory receptor 4D2",
  "term_id": "GO:0005886"
}